{
  "gene": "UniProtKB:Q6ZVD7",
  "term_id": "GO:0005737",
  "term_label": "cytoplasm",
  "gene_symbol": "STOX1",
  "gene_name": "Storkhead-box protein 1"
}